{
  "term_id": "GO:0000298",
  "term_label": "endopolyphosphatase activity",
  "gene": "UniProtKB:O95989",
  "gene_symbol": "NUDT3",
  "gene_name": "Diphosphoinositol polyphosphate phosphohydrolase 1"
}